{
  "term_label": "barbed-end actin filament capping",
  "gene": "UniProtKB:Q6IBS0",
  "term_id": "GO:0051016",
  "gene_symbol": "TWF2",
  "gene_name": "Twinfilin-2"
}